transporter activity [GO:0005215] (molecular function) Definition: Enables the directed movement of substances (such as macromolecules, small molecules, ions) into, out of or within a cell, accross or in between cells. Also known as: carrier Relationships: is a type of molecular_function [GO:0003674] Subtypes: GO:0005319, transmembrane transporter activity [GO:0022857], protein transporter activity [GO:0140318], GO:0160187 Note: Some transporters, such as certain members of the SLC family, are referred to as 'carriers'; however GO uses carrier with a different meaning: a carrier binds to and transports the substance (see GO:0140104 molecular carrier activity), whereas a transporter forms some pore that allows the passing of molecules. Sources: GOC:ai, GOC:dgf Regulation: negatively regulated by negative regulation of transporter activity [GO:0032410]; RO_0002213 by positive regulation of transporter activity [GO:0032411]; regulated by transporter regulator activity [GO:0141108]; RO_0002213 by transporter activator activity [GO:0141109]; negatively regulated by transporter inhibitor activity [GO:0141110]